protein localization involved in acrosome reaction [GO:0060476] (biological process) Also known as: protein localisation involved in acrosome reaction Relationships: is a type of intracellular protein localization [GO:0008104]; is a type of actin filament-based process [GO:0030029]; is part of GO:0007340 Sources: GOC:dph Definition: The actin-based process in which a protein is transported to, or maintained in, a specific location in the sperm as part of the acrosome reaction.